dimethylamine dehydrogenase activity [GO:0047133] (molecular function) Definition: Catalysis of the reaction: electron-transferring flavoprotein + H2O + dimethylamine = reduced electron-transferring flavoprotein + formaldehyde + methylamine. Relationships: is a type of GO:0046997 Also known as: DMADh activity, dimethylamine:electron-transferring flavoprotein oxidoreductase activity Sources: EC:1.5.8.1, MetaCyc:1.5.8.1-RXN